phosphoric diester hydrolase activity [GO:0008081] (molecular function) Relationships: is a type of phosphoric ester hydrolase activity [GO:0042578] Definition: Catalysis of the hydrolysis of a phosphodiester to give a phosphomonoester and a free hydroxyl group. Sources: EC:3.1.4.- Subtypes: cyclic-nucleotide phosphodiesterase activity [GO:0004112], GO:0004528, GO:0004629, GO:0004630, sphingomyelin phosphodiesterase activity [GO:0004767], GO:0008664, GO:0008770, GO:0008889, cardiolipin hydrolase activity [GO:0035755], tyrosyl-RNA phosphodiesterase activity [GO:0036317], protein adenylylhydrolase activity [GO:0044603], 7,8-dihydro-D-neopterin 2',3'-cyclic phosphate phosphodiesterase activity [GO:0044688], serine-ethanolaminephosphate phosphodiesterase activity [GO:0047387], glycerophosphocholine phosphodiesterase activity [GO:0047389], GO:0047390, GO:0047391, CMP-N-acylneuraminate phosphodiesterase activity [GO:0047392], glycerol-1,2-cyclic-phosphate 2-phosphodiesterase activity [GO:0047393], glycerophosphoinositol inositolphosphodiesterase activity [GO:0047394], glycerophosphoinositol glycerophosphodiesterase activity [GO:0047395], dolichylphosphate-glucose phosphodiesterase activity [GO:0047397], dolichylphosphate-mannose phosphodiesterase activity [GO:0047398], GO:0047399, GO:0050290, GPI-mannose ethanolamine phosphate phosphodiesterase activity [GO:0062050], GO:0070259, GO:0070290, cyclic-guanylate-specific phosphodiesterase activity [GO:0071111], phosphodiesterase activity, acting on 3'-phosphoglycolate-terminated DNA strands [GO:0090580], GO:0102561, phosphoribosyl 1,2-cyclic phosphate phosphodiesterase activity [GO:0103043] Also known as: phosphodiesterase